{
  "term_label": "protein serine/threonine kinase activity",
  "gene_name": "Serine_threonine-protein kinase Kist",
  "gene_symbol": "UHMK1",
  "gene": "UniProtKB:Q8TAS1",
  "term_id": "GO:0004674"
}